{
  "term_id": "GO:0030097",
  "gene_name": "Runt-related transcription factor 1",
  "gene_symbol": "RUNX1",
  "term_label": "hemopoiesis",
  "gene": "UniProtKB:Q01196"
}